{
  "gene": "UniProtKB:O94818",
  "gene_symbol": "NOL4",
  "term_id": "UNKNOWN:0002",
  "term_label": "Unknown biological process",
  "gene_name": "Nucleolar protein 4"
}